{
  "gene_symbol": "ARMC6",
  "term_id": "UNKNOWN:0001",
  "gene_name": "Armadillo repeat-containing protein 6",
  "term_label": "Unknown molecular function",
  "gene": "UniProtKB:Q6NXE6"
}